negative regulation of cytoplasmic translational initiation in response to stress [GO:1990625] (biological process) Relationships: is a type of negative regulation of translation in response to stress [GO:0032055]; is a type of negative regulation of translational initiation in response to stress [GO:0032057]; is a type of negative regulation of cytoplasmic translational initiation [GO:1904689]; is a type of GO:1990611 Definition: Any process that stops, prevents or reduces the rate of cytoplasmic translation initiation as a result of a stimulus indicating the organism is under stress. References: PMID:12242291 Sources: GOC:vw